positive regulation of inositol phosphate biosynthetic process [GO:0060732] (BP) Definition: Any process that increases the rate, frequency or extent of inositol phosphate biosynthesis. Inositol phosphate biosynthetic processes are the chemical reactions and pathways resulting in the formation of an inositol phosphate, 1,2,3,4,5,6-cyclohexanehexol, with one or more phosphate groups attached. Relationships: is a type of regulation of inositol phosphate biosynthetic process [GO:0010919]; is a type of positive regulation of carbohydrate metabolic process [GO:0045913]; is a type of positive regulation of phosphate metabolic process [GO:0045937]; is a type of positive regulation of alcohol biosynthetic process [GO:1902932]; positively regulates GO:0032958 Subtypes: positive regulation of inositol trisphosphate biosynthetic process [GO:0032962] Sources: GOC:dph, GOC:tb